{
  "term_label": "adenylate cyclase activity",
  "term_id": "GO:0004016",
  "gene": "UniProtKB:Q08462",
  "gene_symbol": "ADCY2",
  "gene_name": "Adenylate cyclase type 2"
}